{
  "gene_name": "Lysine-specific demethylase PHF2",
  "gene": "UniProtKB:O75151",
  "term_label": "chromatin remodeling",
  "term_id": "GO:0006338",
  "gene_symbol": "PHF2"
}